superior raphe nucleus development [GO:0021725] (biological process) Definition: The process whose specific outcome is the progression of the superior raphe nucleus over time, from its formation to the mature structure. Relationships: is a type of neural nucleus development [GO:0048857]; is part of GO:0021723 References: PMID:19003874 Sources: GOC:cjm, GOC:cls, GOC:curators, GOC:cvs, GOC:dgh Also known as: anterior raphe nucleus development, superior central nucleus development